establishment of myocardial progenitor cell apical/basal polarity [GO:0003316] (biological process) Relationships: is a type of establishment of epithelial cell apical/basal polarity [GO:0045198]; is part of heart rudiment formation [GO:0003315] Definition: The specification and formation of the apicobasal polarity of an myocardial progenitor cell that contributes to the formation of the heart rudiment. Also known as: myocardial progenitor epithelial polarization Sources: GOC:mtg_heart